{
  "term_label": "cytoplasm",
  "gene_symbol": "ANKK1",
  "gene": "UniProtKB:Q8NFD2",
  "gene_name": "Ankyrin repeat and protein kinase domain-containing protein 1",
  "term_id": "GO:0005737"
}